{
  "gene_symbol": "KDM5A",
  "gene_name": "Lysine-specific demethylase 5A",
  "gene": "UniProtKB:P29375",
  "term_id": "GO:0006338",
  "term_label": "chromatin remodeling"
}